{
  "term_label": "mitochondrion",
  "gene": "UniProtKB:A1L188",
  "term_id": "GO:0005739",
  "gene_symbol": "NDUFAF8",
  "gene_name": "NADH dehydrogenase [ubiquinone] 1 alpha subcomplex assembly factor 8"
}